regulation of renal albumin absorption [GO:2000532] (BP) Definition: Any process that modulates the frequency, rate or extent of renal albumin absorption. Sources: GOC:obol, GOC:yaf Relationships: is a type of regulation of renal system process [GO:0098801]; regulates GO:0097018 Subtypes: negative regulation of renal albumin absorption [GO:2000533], positive regulation of renal albumin absorption [GO:2000534]